{
  "gene": "UniProtKB:A0A075B6V7",
  "term_label": "Unknown biological process",
  "gene_name": "T cell receptor alpha joining 26 (Fragment)",
  "gene_symbol": "TRAJ26",
  "term_id": "UNKNOWN:0002"
}